{
  "gene_symbol": "PRKAG3",
  "term_id": "GO:0045722",
  "term_label": "positive regulation of gluconeogenesis",
  "gene": "UniProtKB:Q9UGI9",
  "gene_name": "5'-AMP-activated protein kinase subunit gamma-3"
}